{
  "term_label": "3'-5' DNA helicase activity",
  "term_id": "GO:0043138",
  "gene_symbol": "RECQL5",
  "gene": "UniProtKB:O94762",
  "gene_name": "ATP-dependent DNA helicase Q5"
}